{
  "gene": "UniProtKB:P09619",
  "term_label": "platelet-derived growth factor binding",
  "gene_name": "Platelet-derived growth factor receptor beta",
  "term_id": "GO:0048407",
  "gene_symbol": "PDGFRB"
}